{
  "gene_name": "Putative heat shock protein HSP 90-beta-3",
  "term_id": "GO:0005886",
  "gene": "UniProtKB:Q58FF7",
  "gene_symbol": "HSP90AB3P",
  "term_label": "plasma membrane"
}